trihydroxystilbene synthase activity [GO:0050350] (molecular function) Definition: Catalysis of the reaction: 3 malonyl-CoA + 4-coumaroyl-CoA = 4 CoA + 3,4',5-trihydroxy-stilbene + 4 CO2. Also known as: malonyl-CoA:4-coumaroyl-CoA malonyltransferase (cyclizing), stilbene synthase activity, resveratrol synthase activity Relationships: is a type of acyltransferase activity, transferring groups other than amino-acyl groups [GO:0016747] Sources: EC:2.3.1.95